{
  "gene": "UniProtKB:P28370",
  "term_id": "GO:0045944",
  "gene_symbol": "SMARCA1",
  "term_label": "positive regulation of transcription by RNA polymerase II",
  "gene_name": "Probable global transcription activator SNF2L1"
}